substrate-dependent cell migration, cell attachment to substrate [GO:0006931] (biological process) Definition: The formation of adhesions that stabilize protrusions at the leading edge of a migrating cell; involves integrin activation, clustering, and the recruitment of structural and signaling components to nascent adhesions. Relationships: is a type of cell-substrate adhesion [GO:0031589]; is part of substrate-dependent cell migration [GO:0006929] Also known as: substrate-bound cell migration, cell attachment to substrate References: PMID:11944043, PMID:14657486 Sources: ISBN:0815316194 Regulation: regulated by regulation of substrate-dependent cell migration, cell attachment to substrate [GO:1904235]; negatively regulated by GO:1904236; positively regulated by positive regulation of substrate-dependent cell migration, cell attachment to substrate [GO:1904237]